respiratory chain complex IV assembly [GO:0008535] (biological process) Relationships: is_a cytochrome complex assembly [GO:0017004] References: PMID:32311046 Sources: GOC:jl Subtypes: mitochondrial respiratory chain complex IV assembly [GO:0033617], plasma membrane respiratory chain complex IV assembly [GO:0033618] Also known as: cytochrome c oxidase biogenesis, cytochrome c oxidase complex assembly Definition: The aggregation, arrangement and bonding together of a set of components to form respiratory chain complex IV (also known as cytochrome c oxidase), the terminal member of the respiratory chain of the mitochondrion and some aerobic bacteria. Cytochrome c oxidases are multi-subunit enzymes containing from 13 subunits in the mammalian mitochondrial form to 3-4 subunits in the bacterial forms.